{
  "gene": "UniProtKB:Q9NYT0",
  "gene_symbol": "PLEK2",
  "gene_name": "Pleckstrin-2",
  "term_label": "actin cytoskeleton organization",
  "term_id": "GO:0030036"
}